{
  "gene_name": "Solute carrier family 35 member F1",
  "gene": "UniProtKB:Q5T1Q4",
  "gene_symbol": "SLC35F1",
  "term_id": "UNKNOWN:0001",
  "term_label": "Unknown molecular function"
}